magnetoreception by sensory perception of chemical stimulus [GO:0050977] (biological process) Definition: The series of events required for an organism to receive a chemical stimulus relating to a magnetic field, convert it to a molecular signal, and recognize and characterize the signal. It is believed that organisms such as birds and salamanders use a 'chemical compass': chemical reactions that involve transitions between different spin states can be influenced by magnetic fields and by detecting the different product ratios, these organisms can perceive the direction of the magnetic field. The mechanism by which this is detected is not certain but it may also involve light stimuli. References: PMID:15886990 Sources: GOC:ai, Wikipedia:Magnetoception Also known as: magnetoreception by chemical stimulus, magnetoreception through chemical stimulus, magnetoreception, sensory perception of chemical stimulus, magnetoreception, using chemical stimulus Relationships: is a type of GO:0007606; is_a magnetoreception [GO:0050958]